{
  "gene_symbol": "ADAM8",
  "term_id": "GO:0006508",
  "gene_name": "Disintegrin and metalloproteinase domain-containing protein 8",
  "term_label": "proteolysis",
  "gene": "UniProtKB:P78325"
}